{
  "gene_name": "Heparanase",
  "term_label": "Unknown molecular function",
  "gene_symbol": "HPSE",
  "term_id": "UNKNOWN:0001",
  "gene": "UniProtKB:Q9Y251"
}